{
  "term_id": "GO:0030883",
  "gene_symbol": "CD1B",
  "term_label": "endogenous lipid antigen binding",
  "gene": "UniProtKB:P29016",
  "gene_name": "T-cell surface glycoprotein CD1b"
}